{
  "term_id": "GO:0005886",
  "gene": "UniProtKB:Q13635",
  "gene_name": "Protein patched homolog 1",
  "gene_symbol": "PTCH1",
  "term_label": "plasma membrane"
}